cellular bud neck septin structure [GO:0000399] (cellular component) Definition: Any of a series of septin structures that are localized in the bud neck of a budding fungal cell during the cell cycle. Subtypes: cellular bud neck septin ring [GO:0000144], cellular bud neck septin collar [GO:0032174], GO:0032177 Relationships: is a type of GO:0110165; is part of GO:0005935; is part of GO:0032153 Sources: GOC:krc